{
  "gene_symbol": "RFX5",
  "gene": "UniProtKB:P48382",
  "term_label": "nucleus",
  "gene_name": "DNA-binding protein RFX5",
  "term_id": "GO:0005634"
}